clearance of damaged tissue involved in inflammatory response wound healing [GO:0002247] (biological process) Relationships: is a type of GO:0048771; is part of wound healing involved in inflammatory response [GO:0002246] Sources: GOC:jal, ISBN:0721601871 Definition: The series of events leading to removal of necrotic debris that contribute to an inflammatory response. Also known as: clearance of damaged tissue during inflammatory response